{
  "gene_name": "Cation channel sperm-associated protein 4",
  "gene": "UniProtKB:Q7RTX7",
  "term_label": "voltage-gated calcium channel activity",
  "gene_symbol": "CATSPER4",
  "term_id": "GO:0005245"
}